{
  "term_label": "Unknown molecular function",
  "gene": "UniProtKB:Q96DD7",
  "gene_symbol": "SHISA4",
  "term_id": "UNKNOWN:0001",
  "gene_name": "Protein shisa-4"
}